peptide deformylase activity [GO:0042586] (molecular function) Definition: Catalysis of the reaction: formyl-L-methionyl peptide + H2O = formate + methionyl peptide. Relationships: is a type of hydrolase activity, acting on carbon-nitrogen (but not peptide) bonds, in linear amides [GO:0016811] Sources: EC:3.5.1.88, GOC:jl Also known as: PDF activity, formyl-L-methionyl peptide amidohydrolase activity, polypeptide deformylase activity